{
  "gene": "UniProtKB:O75815",
  "term_id": "UNKNOWN:0003",
  "gene_name": "Breast cancer anti-estrogen resistance protein 3",
  "term_label": "Unknown cellular component",
  "gene_symbol": "BCAR3"
}